RNA translocase activity [GO:0039630] (molecular function) Relationships: is a type of ATP-dependent activity, acting on RNA [GO:0008186] References: PMID:22713318 Sources: GOC:bm Definition: Generating a movement along a single- or double-stranded RNA molecule, driven by ATP hydrolysis. Note: Note that some gene products that possess DNA translocase activity, such as members of the FtsK/SpoIIIE family, can be fixed in place by interactions with other components of the cell; the relative movement between the protein and DNA bound to it results in movement of the DNA within the cell, often across a membrane.